{
  "gene": "UniProtKB:Q9H7P9",
  "term_label": "Unknown cellular component",
  "term_id": "UNKNOWN:0003",
  "gene_symbol": "PLEKHG2",
  "gene_name": "Pleckstrin homology domain-containing family G member 2"
}